{
  "gene_symbol": "ZP4",
  "gene": "UniProtKB:Q12836",
  "term_id": "GO:0007339",
  "term_label": "binding of sperm to zona pellucida",
  "gene_name": "Zona pellucida sperm-binding protein 4"
}